{
  "gene_symbol": "ADCY3",
  "term_id": "GO:0006171",
  "term_label": "cAMP biosynthetic process",
  "gene_name": "Adenylate cyclase type 3",
  "gene": "UniProtKB:O60266"
}